{
  "gene_name": "Transmembrane protein 52",
  "gene_symbol": "TMEM52",
  "gene": "UniProtKB:Q8NDY8",
  "term_label": "Unknown molecular function",
  "term_id": "UNKNOWN:0001"
}